{
  "term_id": "GO:0045892",
  "gene": "UniProtKB:Q8IV76",
  "gene_name": "Circadian clock protein PASD1",
  "gene_symbol": "PASD1",
  "term_label": "negative regulation of DNA-templated transcription"
}